histone H4K20 monomethyltransferase activity [GO:0140944] (molecular function) Note: Note that the residue position corresponds to the canonical human H4 histone (UniProtKB:P02309); this residue is conserved across all eukaryotes. Note that the initiation methionine is cleaved, so the first residue is S1. Definition: Catalysis of the reaction: L-lysyl20-[histone H4] + S-adenosyl-L-methionine = H+ + N6-methyl-L-lysyl20-[histone H4] + S-adenosyl-L-homocysteine. This reaction is the addition of a methyl group to the unmethylated lysine residue at position 20 of histone H4, producing histone H4K20me. Relationships: is a type of histone H4K20 methyltransferase activity [GO:0042799] Also known as: histone H4-K20 methylation, histone H4K20 methylase activity, histone H4K20 methylation, histone H4K20 monomethylation, histone lysine N-monomethyltransferase activity (H4-K20 specific) Sources: RHEA:60344